{
  "term_id": "UNKNOWN:0003",
  "gene_symbol": "ANKS4B",
  "term_label": "Unknown cellular component",
  "gene": "UniProtKB:Q8N8V4",
  "gene_name": "Ankyrin repeat and SAM domain-containing protein 4B"
}